{
  "gene_name": "Deoxyribonuclease-2-alpha",
  "term_label": "deoxyribonuclease II activity",
  "gene": "UniProtKB:O00115",
  "gene_symbol": "DNASE2",
  "term_id": "GO:0004531"
}